oleate hydratase activity [GO:0050151] (molecular function) Sources: EC:4.2.1.53, RHEA:21852 Also known as: (R)-10-hydroxystearate 10-hydro-lyase (oleate-forming), (R)-10-hydroxystearate 10-hydro-lyase activity Relationships: is a type of hydro-lyase activity [GO:0016836] Definition: Catalysis of the reaction: (R)-10-hydroxystearate = H2O + oleate.